{
  "term_label": "respiratory chain complex I",
  "gene_symbol": "NDUFV2",
  "gene": "UniProtKB:P19404",
  "term_id": "GO:0045271",
  "gene_name": "NADH dehydrogenase [ubiquinone] flavoprotein 2, mitochondrial"
}